{
  "gene_name": "DNA-binding protein inhibitor ID-1",
  "term_id": "GO:0003714",
  "gene_symbol": "ID1",
  "gene": "UniProtKB:P41134",
  "term_label": "transcription corepressor activity"
}